{
  "gene": "UniProtKB:O43490",
  "gene_name": "Prominin-1",
  "term_label": "cilium",
  "gene_symbol": "PROM1",
  "term_id": "GO:0005929"
}